{
  "gene_name": "NACHT, LRR and PYD domains-containing protein 7",
  "term_label": "Unknown molecular function",
  "term_id": "UNKNOWN:0001",
  "gene": "UniProtKB:Q8WX94",
  "gene_symbol": "NLRP7"
}